{
  "term_id": "GO:0005886",
  "gene_symbol": "TRBV14",
  "gene_name": "T cell receptor beta variable 14",
  "term_label": "plasma membrane",
  "gene": "UniProtKB:A0A5B0"
}